{
  "gene": "UniProtKB:Q9NPG3",
  "term_id": "UNKNOWN:0001",
  "gene_name": "Ubinuclein-1",
  "gene_symbol": "UBN1",
  "term_label": "Unknown molecular function"
}